catalytic activity, acting on a rRNA [GO:0140102] (MF) Definition: Catalytic activity that acts to modify a ribosomal RNA. Sources: GOC:molecular_function_refactoring, GOC:pdt Relationships: is a type of catalytic activity, acting on RNA [GO:0140098] Subtypes: rRNA methyltransferase activity [GO:0008649], rRNA N-glycosylase activity [GO:0030598], rRNA small subunit aminocarboxypropyltransferase activity [GO:0106388]